{
  "term_label": "Unknown cellular component",
  "gene_symbol": "LOC114841035",
  "term_id": "UNKNOWN:0003",
  "gene": "UniProtKB:A0A494C030",
  "gene_name": "Uncharacterized protein"
}